{
  "gene": "UniProtKB:Q96SB3",
  "term_label": "actin cytoskeleton",
  "gene_name": "Neurabin-2",
  "gene_symbol": "PPP1R9B",
  "term_id": "GO:0015629"
}